negative regulation of amyloid fibril formation [GO:1905907] (biological process) Definition: Any process that stops, prevents or reduces the frequency, rate or extent of amyloid fibril formation. References: PMID:23106396 Sources: GOC:TermGenie, GOC:aruk, GOC:bc, GO_REF:0000058 Relationships: is_a negative regulation of protein metabolic process [GO:0051248]; is a type of GO:1902904; is a type of regulation of amyloid fibril formation [GO:1905906]; negatively regulates GO:1990000 Also known as: down regulation of amyloid fibril formation, down-regulation of amyloid fibril formation, downregulation of amyloid fibril formation, inhibition of amyloid fibril formation, down regulation of amyloid fibril assembly, down regulation of amyloid structure assembly, down regulation of amyloid structure formation, down-regulation of amyloid fibril assembly, down-regulation of amyloid structure assembly, down-regulation of amyloid structure formation, downregulation of amyloid fibril assembly, downregulation of amyloid structure assembly, downregulation of amyloid structure formation, inhibition of amyloid fibril assembly, inhibition of amyloid structure assembly, inhibition of amyloid structure formation, negative regulation of amyloid fibril assembly, negative regulation of amyloid structure assembly, negative regulation of amyloid structure formation Note: Although deposition of amyloid fibrils is associated with diseases, e.g. Alzheimer's disease, amyloid formation is a normal process. Disease occurs when the balance between amyloid formation and clearance is disrupted (reviewed e.g. in PMID:29654159 and PMID:28937655). An example of a normal amyloid complex is composed of human RIP1 and RIP3 kinases (PMID:22817896).